5-hydroxymethyl-dUMP N-hydrolase activity [GO:0070694] (molecular function) Definition: Catalysis of the reaction: 5-hydroxymethyl-dUMP + H2O = 2-deoxy-D-ribose 5-phosphate + 5-hydroxymethyluracil. References: PMID:17234634 Sources: RHEA:77099 Also known as: deoxynucleoside 5'-monophosphate N-glycosidase activity Relationships: is_a hydrolase activity, hydrolyzing N-glycosyl compounds [GO:0016799]